glycerol-3-phosphate oxidase activity [GO:0004369] (molecular function) Definition: Catalysis of the reaction: sn-glycerol 3-phosphate + O2 = glycerone phosphate + H2O2. Relationships: is a type of oxidoreductase activity, acting on the CH-OH group of donors, oxygen as acceptor [GO:0016899] Sources: EC:1.1.3.21, RHEA:18369 Also known as: L-alpha-glycerol-3-phosphate oxidase activity, L-alpha-glycerophosphate oxidase activity, alpha-glycerophosphate oxidase activity, glycerol phosphate oxidase activity, glycerol-1-phosphate oxidase activity, sn-glycerol-3-phosphate:oxygen 2-oxidoreductase activity